phosphatidylcholine biosynthetic process [GO:0006656] (biological process) Subtypes: GO:0006657, phosphatidylcholine biosynthesis from phosphoryl-ethanolamine via N-dimethylethanolamine phosphate and CDP-choline [GO:0070832], phosphatidylcholine biosynthesis from phosphoryl-ethanolamine via CDP-N-methylethanolamine [GO:0070833], GO:0070834, phosphatidylcholine biosynthesis from phosphatidylethanolamine [GO:0090638], phosphatidylcholine biosynthesis from choline and CDP-diacylglycerol [GO:0090639], phosphatidylcholine biosynthesis from sn-glycero-3-phosphocholine [GO:0090640] Sources: ISBN:0198506732 Regulation: regulated by GO:2001245; negatively regulated by negative regulation of phosphatidylcholine biosynthetic process [GO:2001246]; positively regulated by GO:2001247 Also known as: phosphatidylcholine anabolism, phosphatidylcholine biosynthesis, phosphatidylcholine formation, phosphatidylcholine synthesis Relationships: is a type of phosphatidylcholine metabolic process [GO:0046470]; is a type of glycerophospholipid biosynthetic process [GO:0046474] Definition: The chemical reactions and pathways resulting in the formation of phosphatidylcholines, any of a class of glycerophospholipids in which the phosphatidyl group is esterified to the hydroxyl group of choline.